{
  "gene": "UniProtKB:Q3LI59",
  "term_id": "UNKNOWN:0003",
  "gene_name": "Keratin-associated protein 21-2",
  "gene_symbol": "KRTAP21-2",
  "term_label": "Unknown cellular component"
}